{
  "gene_name": "SLIT-ROBO Rho GTPase-activating protein 2",
  "gene_symbol": "SRGAP2",
  "term_label": "dendritic spine",
  "term_id": "GO:0043197",
  "gene": "UniProtKB:O75044"
}